{
  "gene": "UniProtKB:Q99678",
  "gene_symbol": "GPR20",
  "term_label": "plasma membrane",
  "term_id": "GO:0005886",
  "gene_name": "G-protein coupled receptor 20"
}